{
  "gene_name": "Zinc finger protein 329",
  "term_id": "GO:0006357",
  "term_label": "regulation of transcription by RNA polymerase II",
  "gene": "UniProtKB:Q86UD4",
  "gene_symbol": "ZNF329"
}